catalytic activity, acting on DNA [GO:0140097] (molecular function) Subtypes: GO:0000150, DNA ligase activity [GO:0003909], GO:0003913, DNA topoisomerase activity [GO:0003916], DNA nuclease activity [GO:0004536], transposase activity [GO:0004803], ATP-dependent activity, acting on DNA [GO:0008094], integrase activity [GO:0008907], DNA-methyltransferase activity [GO:0009008], GO:0019104, DNA alpha-glucosyltransferase activity [GO:0033820], DNA beta-glucosyltransferase activity [GO:0033821], DNA-deoxyinosine glycosylase activity [GO:0033958], deoxyribodipyrimidine endonucleosidase activity [GO:0033959], DNA polymerase activity [GO:0034061], GO:0035514, site-specific telomere resolvase activity [GO:0043336], dATP(dGTP)-DNA purinetransferase activity [GO:0047839], GO:0051575, GO:0061775, tyrosyl-DNA phosphodiesterase activity [GO:0070259], DNA 5-methylcytosine dioxygenase activity [GO:0070579], phosphodiesterase activity, acting on 3'-phosphoglycolate-terminated DNA strands [GO:0090580], 3'-deoxyribose phosphate lyase activity [GO:0106334], cohesin unloader activity [GO:0140670], DNA/DNA annealing activity [GO:1990814] Definition: Catalytic activity that acts to modify DNA. Relationships: is a type of catalytic activity, acting on a nucleic acid [GO:0140640] Sources: GOC:molecular_function_refactoring, GOC:pdt